{
  "gene_symbol": "EPN1",
  "gene": "UniProtKB:Q9Y6I3",
  "term_id": "GO:0005768",
  "term_label": "endosome",
  "gene_name": "Epsin-1"
}